{
  "gene_symbol": "PARD6G",
  "term_label": "Unknown molecular function",
  "gene": "UniProtKB:Q9BYG4",
  "term_id": "UNKNOWN:0001",
  "gene_name": "Partitioning defective 6 homolog gamma"
}